{
  "gene_symbol": "HCRT",
  "term_label": "temperature homeostasis",
  "gene": "UniProtKB:O43612",
  "gene_name": "Hypocretin neuropeptide precursor",
  "term_id": "GO:0001659"
}